{
  "term_label": "Unknown molecular function",
  "gene": "UniProtKB:Q9NWX5",
  "gene_symbol": "ASB6",
  "gene_name": "Ankyrin repeat and SOCS box protein 6",
  "term_id": "UNKNOWN:0001"
}